{
  "gene_symbol": "RYBP",
  "gene": "UniProtKB:Q8N488",
  "term_label": "transcription coregulator activity",
  "gene_name": "RING1 and YY1-binding protein",
  "term_id": "GO:0003712"
}